ammonium transmembrane transport [GO:0072488] (biological process) Note: Note that this term is not intended for use in annotating lateral movement within membranes. Relationships: is a type of transmembrane transport [GO:0055085]; is a type of nitrogen compound transport [GO:0071705] Subtypes: ammonium import across plasma membrane [GO:0140157] Definition: The process in which ammonium is transported across a membrane. Ammonium is the cation NH4+. Also known as: ammonia transport, ammonium transport, ammonium membrane transport Sources: GOC:mah